negative regulation of complement activation, alternative pathway [GO:0045957] (biological process) Definition: Any process that stops, prevents, or reduces the frequency, rate or extent of complement activation by the alternative pathway. Also known as: down regulation of complement activation, alternative pathway, down-regulation of complement activation, alternative pathway, downregulation of complement activation, alternative pathway, negative regulation of complement cascade, alternative pathway, inhibition of complement activation, alternative pathway Sources: GOC:go_curators Relationships: is a type of GO:0030451; is a type of negative regulation of innate immune response [GO:0045824]; is a type of GO:0045916; negatively regulates GO:0006957